very-long-chain fatty acyl-CoA oxidase activity [GO:0044535] (molecular function) Note: While there is not universal consensus on the lengths of short-, medium-, long- and very-long-chain fatty acids, the GO uses the definitions in ChEBI (see CHEBI:26666, CHEBI:59554, CHEBI:15904 and CHEBI:27283). References: PMID:17458872 Sources: RHEA:78847 Also known as: VLC fatty-acyl-CoA oxidase activity, very long chain fatty-acyl-CoA oxidase activity, very-long-chain acyl-CoA oxidase activity Relationships: is a type of acyl-CoA oxidase activity [GO:0003997] Definition: Catalysis of the reaction: a very-long-chain 2,3-saturated fatty acyl-CoA + O2 = a very-long-chain (2E)-enoyl-CoA + H2O2.